Wnt receptor catabolic process [GO:0038018] (biological process) References: PMID:19643732 Sources: GOC:BHF, GOC:rl, GOC:signaling Also known as: Wnt receptor breakdown, Wnt receptor catabolism, negative regulation of Wnt receptor signaling pathway by Wnt receptor degradation, Frizzled degradation, Wnt receptor degradation Definition: The chemical reactions and pathways resulting in the breakdown of a Wnt receptor. Internalized Wnt receptors can be recycled to the plasma membrane or sorted to lysosomes for protein degradation. Relationships: is a type of receptor catabolic process [GO:0032801]; is part of negative regulation of Wnt signaling pathway [GO:0030178]